negative regulation of auxin metabolic process [GO:0090356] (biological process) Relationships: is a type of GO:0032351; is a type of regulation of auxin metabolic process [GO:0090354]; negatively regulates auxin metabolic process [GO:0009850] Sources: GOC:tb Subtypes: negative regulation of indoleacetic acid biosynthetic process via tryptophan [GO:1901997] Definition: Any process that decreases the frequency, rate or extent of the chemical reactions and pathways involving auxins, plant hormones that regulate aspects of plant growth. Also known as: negative regulation of auxin metabolism